{
  "gene_symbol": "NCBP2L",
  "gene_name": "Nuclear cap-binding protein subunit 2-like",
  "term_label": "RNA cap binding",
  "gene": "UniProtKB:A6PVI3",
  "term_id": "GO:0000339"
}